regulation of dendritic cell antigen processing and presentation [GO:0002604] (biological process) Subtypes: GO:0002605, positive regulation of dendritic cell antigen processing and presentation [GO:0002606], regulation of myeloid dendritic cell antigen processing and presentation [GO:0002607], GO:0002610 Definition: Any process that modulates the frequency, rate, or extent of dendritic cell antigen processing and presentation. Sources: GOC:add Relationships: is a type of regulation of antigen processing and presentation [GO:0002577]; regulates GO:0002468